phosphate butyryltransferase activity [GO:0050182] (molecular function) Also known as: butanoyl-CoA:phosphate butanoyltransferase activity, phosphotransbutyrylase activity Sources: EC:2.3.1.19, RHEA:20892 Relationships: is a type of acyltransferase activity, transferring groups other than amino-acyl groups [GO:0016747] Definition: Catalysis of the reaction: butanoyl-CoA + phosphate = butanoyl phosphate + CoA.